phosphatidylinositol 3-kinase complex [GO:0005942] (cellular component) Definition: A protein complex capable of phosphatidylinositol 3-kinase activity and containing subunits of any phosphatidylinositol 3-kinase (PI3K) enzyme. These complexes are divided in three classes (called I, II and III) that differ for their presence across taxonomic groups and for the type of their constituents. Catalytic subunits of phosphatidylinositol 3-kinase enzymes are present in all 3 classes; regulatory subunits of phosphatidylinositol 3-kinase enzymes are present in classes I and III; adaptor proteins have been observed in class II complexes and may be present in other classes too. Note: For discussion of membrane association, please see https://sourceforge.net/p/geneontology/ontology-requests/11559/ Subtypes: phosphatidylinositol 3-kinase complex, class III [GO:0035032], phosphatidylinositol 3-kinase complex, class I [GO:0097651], phosphatidylinositol 3-kinase complex, class II [GO:0097652] Relationships: is a type of GO:0061695; is a type of GO:0098796; is part of GO:0019898 References: PMID:24587488 Sources: GOC:bf Also known as: 1-phosphatidylinositol 3-kinase complex, PI3K complex, phosphoinositide 3-kinase complex, PI3-kinase p85-subunit alpha- PI3-kinase p110 complex, PIK3C3-PIK3R4 complex, PIK3CA-PIK3R1 complex